{
  "gene_symbol": "NXPE1",
  "term_id": "UNKNOWN:0002",
  "gene_name": "NXPE family member 1",
  "term_label": "Unknown biological process",
  "gene": "UniProtKB:Q8N323"
}